{
  "gene": "UniProtKB:Q07444",
  "term_id": "GO:0045954",
  "gene_symbol": "KLRC3",
  "gene_name": "NKG2-E type II integral membrane protein",
  "term_label": "positive regulation of natural killer cell mediated cytotoxicity"
}